{
  "term_id": "UNKNOWN:0003",
  "gene": "UniProtKB:A6NI87",
  "term_label": "Unknown cellular component",
  "gene_symbol": "CBY3",
  "gene_name": "Protein chibby homolog 3"
}